{
  "gene_symbol": "RAB39B",
  "gene": "UniProtKB:Q96DA2",
  "term_id": "GO:0031489",
  "term_label": "myosin V binding",
  "gene_name": "Ras-related protein Rab-39B"
}